mitochondrial outer membrane permeabilization involved in programmed cell death [GO:1902686] (biological process) Definition: The process by which the mitochondrial outer membrane becomes permeable to the passing of proteins and other molecules from the intermembrane space to the cytosol as part of a programmed cell death process. References: PMID:20151314 Sources: GOC:TermGenie, GOC:mtg_apoptosis, GOC:pg, GO_REF:0000060 Also known as: mitochondrial outer membrane permeabilization during programmed cell death, mitochondrion outer membrane permeabilization involved in programmed cell death, positive regulation of mitochondrial membrane permeability involved in PCD, positive regulation of mitochondrial membrane permeability involved in programmed cell death, positive regulation of transport across mitochondrial membrane involved in PCD, positive regulation of transport across mitochondrial membrane involved in programmed cell death, MPT involved in PCD, MPT involved in caspase-independent cell death, MPT involved in non-apoptotic programmed cell death, MPT involved in nonapoptotic programmed cell death, MPT involved in programmed cell death, mitochondrial membrane permeability transition involved in PCD, mitochondrial membrane permeability transition involved in caspase-independent cell death, mitochondrial membrane permeability transition involved in non-apoptotic programmed cell death, mitochondrial membrane permeability transition involved in nonapoptotic programmed cell death, mitochondrial membrane permeability transition involved in programmed cell death, mitochondrial membrane permeabilization involved in PCD, mitochondrial membrane permeabilization involved in caspase-independent cell death, mitochondrial membrane permeabilization involved in non-apoptotic programmed cell death, mitochondrial membrane permeabilization involved in nonapoptotic programmed cell death, mitochondrial membrane permeabilization involved in programmed cell death, mitochondrial permeability transition involved in PCD, mitochondrial permeability transition involved in caspase-independent cell death, mitochondrial permeability transition involved in non-apoptotic programmed cell death, mitochondrial permeability transition involved in nonapoptotic programmed cell death, mitochondrial permeability transition involved in programmed cell death, positive regulation of mitochondrial membrane permeability involved in caspase-independent cell death, positive regulation of mitochondrial membrane permeability involved in non-apoptotic programmed cell death, positive regulation of mitochondrial membrane permeability involved in nonapoptotic programmed cell death, positive regulation of transport across mitochondrial membrane involved in caspase-independent cell death, positive regulation of transport across mitochondrial membrane involved in non-apoptotic programmed cell death, positive regulation of transport across mitochondrial membrane involved in nonapoptotic programmed cell death, MPT involved in caspase-independent apoptosis, MPT involved in regulated cell death, mitochondrial membrane permeability transition involved in caspase-independent apoptosis, mitochondrial membrane permeability transition involved in regulated cell death, mitochondrial membrane permeabilization involved in caspase-independent apoptosis, mitochondrial membrane permeabilization involved in regulated cell death, mitochondrial permeability transition involved in caspase-independent apoptosis, mitochondrial permeability transition involved in regulated cell death, positive regulation of mitochondrial membrane permeability involved in caspase-independent apoptosis, positive regulation of mitochondrial membrane permeability involved in regulated cell death, positive regulation of transport across mitochondrial membrane involved in caspase-independent apoptosis, positive regulation of transport across mitochondrial membrane involved in regulated cell death Relationships: is a type of positive regulation of mitochondrial membrane permeability [GO:0035794]; is part of programmed cell death [GO:0012501] Subtypes: positive regulation of mitochondrial membrane permeability involved in apoptotic process [GO:1902110]